negative regulation of naphtho-gamma-pyrone biosynthetic process [GO:1900847] (biological process) Also known as: down regulation of naphtho-gamma-pyrone biosynthetic process, down-regulation of naphtho-gamma-pyrone biosynthetic process, downregulation of naphtho-gamma-pyrone biosynthetic process, inhibition of naphtho-gamma-pyrone biosynthetic process Definition: Any process that stops, prevents or reduces the frequency, rate or extent of naphtho-gamma-pyrone biosynthetic process. Relationships: is a type of GO:0009890; is a type of negative regulation of small molecule metabolic process [GO:0062014]; is_a regulation of naphtho-gamma-pyrone biosynthetic process [GO:1900846]; RO_0002212 naphtho-gamma-pyrone biosynthetic process [GO:1900787] Sources: GOC:TermGenie, GOC:di